{
  "gene_name": "Adipogenin",
  "term_id": "UNKNOWN:0001",
  "gene_symbol": "ADIG",
  "gene": "UniProtKB:Q0VDE8",
  "term_label": "Unknown molecular function"
}